DNA topoisomerase type II (double strand cut, ATP-hydrolyzing) activity [GO:0003918] (molecular function) References: PMID:8811192 Also known as: deoxyribonucleate topoisomerase, deoxyribonucleic topoisomerase activity, topoisomerase, DNA topoisomerase type II activity, DNA topoisomerase II, DNA topoisomerase II activity, DNA topoisomerase IV activity, topoisomerase II, DNA topoisomerase (ATP-hydrolysing), type II DNA topoisomerase activity Regulation: negatively regulated by DNA topoisomerase type II (double strand cut, ATP-hydrolyzing) inhibitor activity [GO:0008657]; RO_0002211 by DNA topoisomerase type II (double strand cut, ATP-hydrolyzing) regulator activity [GO:0072586]; positively regulated by DNA topoisomerase type II (double strand cut, ATP-hydrolyzing) activator activity [GO:0072587]; positively regulated by GO:2000373 Definition: Catalysis of a DNA topological transformation by transiently cleaving a pair of complementary DNA strands to form a gate through which a second double-stranded DNA segment is passed, after which the severed strands in the first DNA segment are rejoined, driven by ATP hydrolysis. The enzyme changes the linking number in multiples of 2. Relationships: is a type of GO:0003916; is a type of ATP-dependent activity, acting on DNA [GO:0008094] Subtypes: DNA negative supercoiling activity [GO:0034335]